{
  "term_id": "GO:0006508",
  "term_label": "proteolysis",
  "gene_symbol": "CAPN8",
  "gene": "UniProtKB:A6NHC0",
  "gene_name": "Calpain-8"
}